commitment complex [GO:0000243] (cellular component) Definition: A spliceosomal complex that is formed by association of the U1 snRNP with the 5' splice site of an unspliced intron in an RNA transcript. References: PMID:9150140 Sources: GOC:krc, ISBN:0879695897 Relationships: is a type of U2-type spliceosomal complex [GO:0005684]; has part U1 snRNP [GO:0005685] Also known as: mammalian spliceosomal E complex, mammalian spliceosomal complex E, yeast spliceosomal complex CC